podocyte foot [GO:0098846] (cellular component) Also known as: pedicel, podocyte foot process, secondary podocyte projection Relationships: is a type of plasma membrane bounded cell projection [GO:0120025] References: PMID:25324828 Definition: A cell projection of a podocyte (glomerular visceral epithelial cell) forming a foot-like structure projecting from a podocyte primary projection, that wraps around capillaries of a renal glomerulus. Adjacent feet (pedicels) interdigitate, leaving thin filtration slits between them, which are covered by slit diaphragms.